{
  "term_label": "plasma membrane",
  "gene_symbol": "EPHA10",
  "gene": "UniProtKB:Q5JZY3",
  "term_id": "GO:0005886",
  "gene_name": "Ephrin type-A receptor 10"
}